{
  "term_label": "Unknown biological process",
  "gene_name": "Protein FRG2",
  "gene": "UniProtKB:Q64ET8",
  "term_id": "UNKNOWN:0002",
  "gene_symbol": "FRG2"
}